{
  "gene": "UniProtKB:O75452",
  "gene_symbol": "RDH16",
  "term_id": "GO:0004745",
  "term_label": "all-trans-retinol dehydrogenase (NAD+) activity",
  "gene_name": "Retinol dehydrogenase 16"
}